{
  "term_label": "spliceosomal tri-snRNP complex assembly",
  "gene_symbol": "PRPF6",
  "gene": "UniProtKB:O94906",
  "gene_name": "Pre-mRNA-processing factor 6",
  "term_id": "GO:0000244"
}